glutamate-tRNA(Gln) ligase activity [GO:0050561] (molecular function) Sources: EC:6.1.1.24, MetaCyc:6.1.1.24-RXN Relationships: is a type of aminoacyl-tRNA ligase activity [GO:0004812] Also known as: glutamate-tRNAGln ligase activity, L-glutamate:tRNAGlx ligase (AMP-forming), nondiscriminating glutamyl-tRNA synthetase activity Definition: Catalysis of the reaction: tRNA(Glx) + L-glutamate + ATP = glutamyl-tRNA(Glx) + diphosphate + AMP.